{
  "gene_name": "Homeobox protein Nkx-2.3",
  "term_label": "nucleus",
  "term_id": "GO:0005634",
  "gene": "UniProtKB:Q8TAU0",
  "gene_symbol": "NKX2-3"
}